{
  "gene_symbol": "DCSTAMP",
  "gene": "UniProtKB:Q9H295",
  "term_label": "Unknown molecular function",
  "term_id": "UNKNOWN:0001",
  "gene_name": "Dendritic cell-specific transmembrane protein"
}